{
  "gene_symbol": "IGKV1D-43",
  "gene": "UniProtKB:A0A0B4J1Z2",
  "term_label": "Unknown molecular function",
  "gene_name": "Immunoglobulin kappa variable 1D-43",
  "term_id": "UNKNOWN:0001"
}